nuclear exosome targeting complex [GO:0062141] (cellular component) References: PMID:21855801, PMID:29844170 Relationships: is_a nuclear protein-containing complex [GO:0140513] Also known as: NEXT complex Definition: A protein-containing complex that functions with the RNA exosome and contributes to the degradation of abberant transcripts.